{
  "term_label": "ERAD pathway",
  "gene_symbol": "RNF145",
  "gene_name": "RING finger protein 145",
  "gene": "UniProtKB:Q96MT1",
  "term_id": "GO:0036503"
}